geranyl-diphosphate cyclase activity [GO:0047926] (molecular function) Relationships: is a type of GO:0009975; is a type of intramolecular lyase activity [GO:0016872] References: PMID:42357 Sources: RHEA:18209 Also known as: (+)-bornyl-diphosphate lyase (decyclizing), (+)-bornylpyrophosphate cyclase activity, bornyl diphosphate synthase activity, bornyl pyrophosphate synthase activity, bornyl pyrophosphate synthetase activity Definition: Catalysis of the reaction: geranyl diphosphate = (2S)-bornyl diphosphate.